regulation of telomere maintenance via recombination [GO:0032207] (biological process) Relationships: is a type of regulation of mitotic recombination [GO:0000019]; is_a GO:0032204; is a type of regulation of DNA recombination at telomere [GO:0072695]; regulates telomere maintenance via recombination [GO:0000722] Sources: GOC:mah Definition: Any process that modulates the frequency, rate or extent of a recombinational process involved in the maintenance of proper telomeric length. Subtypes: negative regulation of telomere maintenance via recombination [GO:0032208], positive regulation of telomere maintenance via recombination [GO:0032209]